perithecium development [GO:0120165] (biological process) References: PMID:125266, PMID:19547974, PMID:20739093, PMID:25311923 Sources: DOI:10.1007/978-3-642-00286-1_2 Subtypes: GO:0106154 Definition: The process whose specific outcome is the progression of a perithecium over time, from its formation to the mature structure. Peritheicum is a flask-shaped fruiting body of certain molds and ascomycetous fungi having a pore for the escape of spores. In the ascomycetous fungi such as Neurospora crassa and Sordaria macrospora, these perithecia are formed in the sexual phase and they discharge ascospores through the ostiolum at the tip of the perithecial neck. Relationships: is a type of reproductive fruiting body development [GO:0030582]